{
  "gene_name": "G-protein coupled receptor 42",
  "term_id": "UNKNOWN:0002",
  "term_label": "Unknown biological process",
  "gene_symbol": "GPR42",
  "gene": "UniProtKB:O15529"
}